{
  "gene_symbol": "RTL6",
  "term_id": "UNKNOWN:0001",
  "gene_name": "Retrotransposon Gag-like protein 6",
  "term_label": "Unknown molecular function",
  "gene": "UniProtKB:Q6ICC9"
}